{
  "term_label": "regulation of protein stability",
  "gene_name": "Ubiquitin carboxyl-terminal hydrolase 17-like protein 20",
  "gene": "UniProtKB:D6RJB6",
  "term_id": "GO:0031647",
  "gene_symbol": "USP17L20"
}